{
  "term_label": "Unknown molecular function",
  "gene_name": "Mitochondrial fission regulator 1-like",
  "gene_symbol": "MTFR1L",
  "gene": "UniProtKB:Q9H019",
  "term_id": "UNKNOWN:0001"
}